{
  "gene": "UniProtKB:Q8WXK1",
  "term_label": "Unknown biological process",
  "gene_symbol": "ASB15",
  "term_id": "UNKNOWN:0002",
  "gene_name": "Ankyrin repeat and SOCS box protein 15"
}